{
  "term_id": "UNKNOWN:0002",
  "gene": "UniProtKB:Q96IL0",
  "gene_name": "Cytochrome c oxidase assembly factor 8",
  "term_label": "Unknown biological process",
  "gene_symbol": "COA8"
}